{
  "gene": "UniProtKB:O75129",
  "gene_name": "Astrotactin-2",
  "term_label": "neuron cell-cell adhesion",
  "gene_symbol": "ASTN2",
  "term_id": "GO:0007158"
}